{
  "term_id": "GO:0005764",
  "gene_symbol": "GALC",
  "gene": "UniProtKB:P54803",
  "gene_name": "Galactocerebrosidase",
  "term_label": "lysosome"
}